cytokinin catabolic process [GO:0009823] (biological process) Relationships: is a type of cytokinin metabolic process [GO:0009690]; is a type of GO:0042447 Subtypes: isopentenyl adenine catabolic process [GO:0034266], discadenine catabolic process [GO:0034269] Definition: The chemical reactions and pathways resulting in the breakdown of cytokinins, a class of adenine-derived compounds that can function in plants as plant growth regulators. Also known as: cytokinin breakdown, cytokinin catabolism, cytokinin degradation Sources: GOC:lr